serotonin biosynthetic process [GO:0042427] (BP) Relationships: is a type of serotonin metabolic process [GO:0042428]; is_a indole-containing compound biosynthetic process [GO:0042435]; is_a phenol-containing compound biosynthetic process [GO:0046189]; is a type of primary amino compound biosynthetic process [GO:1901162] Sources: GOC:jl, ISBN:0198506732 Subtypes: serotonin biosynthetic process from tryptophan [GO:0006587] Regulation: regulated by regulation of serotonin biosynthetic process [GO:1905627]; negatively regulated by negative regulation of serotonin biosynthetic process [GO:1905628]; positively regulated by GO:1905629 Also known as: serotonin anabolism, serotonin biosynthesis, serotonin formation, serotonin synthesis Definition: The chemical reactions and pathways resulting in the formation of serotonin (5-hydroxytryptamine), a monoamine neurotransmitter occurring in the peripheral and central nervous systems, also having hormonal properties.